{
  "term_label": "transmembrane-ephrin receptor activity",
  "gene": "UniProtKB:P54762",
  "gene_name": "Ephrin type-B receptor 1",
  "gene_symbol": "EPHB1",
  "term_id": "GO:0005005"
}